{
  "gene": "UniProtKB:Q9NZT1",
  "term_id": "GO:0030234",
  "gene_name": "Calmodulin-like protein 5",
  "term_label": "enzyme regulator activity",
  "gene_symbol": "CALML5"
}